{
  "term_label": "odorant binding",
  "gene_symbol": "OR8D2",
  "gene": "UniProtKB:Q9GZM6",
  "term_id": "GO:0005549",
  "gene_name": "Olfactory receptor 8D2"
}